{
  "gene_symbol": "GGA1",
  "gene": "UniProtKB:Q9UJY5",
  "gene_name": "ADP-ribosylation factor-binding protein GGA1",
  "term_label": "protein localization to cell surface",
  "term_id": "GO:0034394"
}